{
  "term_id": "GO:0005219",
  "gene_symbol": "RYR3",
  "gene_name": "Ryanodine receptor 3",
  "term_label": "ryanodine-sensitive calcium-release channel activity",
  "gene": "UniProtKB:Q15413"
}